symbiont-mediated killing of host cell [GO:0001907] (biological process) Subtypes: symbiont-mediated cytolysis of host cell [GO:0001897], killing by virus of host cell during superinfection exclusion [GO:0039634], killing by virus of host cell by post-segregational killing [GO:0044696], symbiont-mediated activation of host apoptosis [GO:0052151] Also known as: killing by symbiont of host cells, pathogenesis Relationships: is_a killing of cells of another organism [GO:0031640]; is a type of biological process involved in interaction with host [GO:0051701] References: PMID:11123917, PMID:22992735, PMID:23230295, PMID:26633512 Sources: GOC:add Definition: A process mediated by a symbiont that results in the death of a cell in the host organism. The host is defined as the larger of the organisms involved in a symbiotic interaction.